{
  "gene": "UniProtKB:Q12926",
  "term_label": "Unknown biological process",
  "gene_name": "ELAV-like protein 2",
  "gene_symbol": "ELAVL2",
  "term_id": "UNKNOWN:0002"
}